quinol-cytochrome-c reductase activity [GO:0008121] (molecular function) Definition: Enables the transfer of a solute or solutes from one side of a membrane to the other according to the reaction: a quinol + 2 Fe(III)-cytochrome c = a quinone + 2 Fe(II)-cytochrome c + 2 H+(out). Sources: RHEA:11484 Also known as: cytochrome, complex III (mitochondrial electron transport) activity, cytochrome a, cytochrome a3/copper complex, cytochrome b562, cytochrome b566, cytochrome c1, soluble cytochrome b562, ubiquinol-cytochrome-c reductase activity, electron transporter, transferring electrons within CoQH2-cytochrome c reductase complex activity, electron transporter, transferring electrons within cytochrome c oxidase complex activity, mitochondrial electron transport complex III, ubiquinol-cytochrome c oxidoreductase activity, ubiquinol-cytochrome c-2 oxidoreductase activity, ubiquinol-cytochrome c1 oxidoreductase activity, ubiquinol-cytochrome c2 reductase activity, ubiquinol:ferricytochrome-c oxidoreductase activity, ubiquinone--cytochrome-c oxidoreductase activity, ubiquinone-cytochrome c oxidoreductase activity, ubiquinone-cytochrome c reductase activity Relationships: is a type of electron transfer activity [GO:0009055]; is a type of proton transmembrane transporter activity [GO:0015078]; is a type of oxidoreduction-driven active transmembrane transporter activity [GO:0015453]; is a type of GO:0022853; has part oxidoreductase activity, acting on diphenols and related substances as donors [GO:0016679]